{
  "term_id": "GO:0005634",
  "gene_name": "Zinc finger protein 551",
  "gene": "UniProtKB:Q7Z340",
  "gene_symbol": "ZNF551",
  "term_label": "nucleus"
}